{
  "term_id": "GO:1990072",
  "gene_name": "Trafficking protein particle complex subunit 5",
  "gene": "UniProtKB:Q8IUR0",
  "gene_symbol": "TRAPPC5",
  "term_label": "TRAPPIII protein complex"
}